{
  "gene_name": "Retinal guanylyl cyclase 1",
  "gene": "UniProtKB:Q02846",
  "term_id": "GO:0006182",
  "term_label": "cGMP biosynthetic process",
  "gene_symbol": "GUCY2D"
}